{
  "term_id": "GO:0003755",
  "term_label": "peptidyl-prolyl cis-trans isomerase activity",
  "gene_symbol": "PIN1",
  "gene": "UniProtKB:Q13526",
  "gene_name": "Peptidyl-prolyl cis-trans isomerase NIMA-interacting 1"
}